meiotic sister chromatid cohesion involved in meiosis I [GO:0010789] (BP) Relationships: is a type of meiotic sister chromatid cohesion [GO:0051177] Sources: GOC:dph, GOC:tb Definition: The cell cycle process in which sister chromatids of a replicated chromosome are joined along the entire length of the chromosome during meiosis I.